{
  "gene_symbol": "AVPR1B",
  "gene_name": "Vasopressin V1b receptor",
  "term_label": "G protein-coupled receptor signaling pathway",
  "term_id": "GO:0007186",
  "gene": "UniProtKB:P47901"
}